negative regulation of pupariation [GO:0106024] (biological process) Relationships: is a type of GO:0048581; is a type of GO:0106023; negatively regulates pupariation [GO:0035073] References: PMID:26510564 Definition: Any process that stops, prevents or reduces the rate of onset of pupariation.